{
  "term_id": "GO:0005886",
  "term_label": "plasma membrane",
  "gene": "UniProtKB:A0A1B0GX51",
  "gene_name": "T cell receptor beta variable 7-8",
  "gene_symbol": "TRBV7-8"
}